{
  "gene_name": "Small nuclear ribonucleoprotein-associated proteins B and B'",
  "term_label": "U1 snRNP",
  "gene_symbol": "SNRPB",
  "gene": "UniProtKB:P14678",
  "term_id": "GO:0005685"
}